{
  "term_id": "GO:0071221",
  "gene_symbol": "TLR10",
  "gene_name": "Toll-like receptor 10",
  "term_label": "cellular response to bacterial lipopeptide",
  "gene": "UniProtKB:Q9BXR5"
}